negative regulation of protein tetramerization [GO:1901091] (biological process) Definition: Any process that stops, prevents or reduces the frequency, rate or extent of protein tetramerization. Sources: GOC:TermGenie, GOC:pm Also known as: down regulation of protein tetramer assembly, down regulation of protein tetramer biosynthesis, down regulation of protein tetramer biosynthetic process, down regulation of protein tetramer formation, down regulation of protein tetramerization, down-regulation of protein tetramer assembly, down-regulation of protein tetramer biosynthesis, down-regulation of protein tetramer biosynthetic process, down-regulation of protein tetramer formation, down-regulation of protein tetramerization, downregulation of protein tetramer assembly, downregulation of protein tetramer biosynthesis, downregulation of protein tetramer biosynthetic process, downregulation of protein tetramer formation, downregulation of protein tetramerization, negative regulation of protein tetramer assembly, negative regulation of protein tetramer biosynthesis, negative regulation of protein tetramer biosynthetic process, negative regulation of protein tetramer formation, inhibition of protein tetramer assembly, inhibition of protein tetramer biosynthesis, inhibition of protein tetramer biosynthetic process, inhibition of protein tetramer formation, inhibition of protein tetramerization Relationships: is a type of negative regulation of protein oligomerization [GO:0032460]; is a type of regulation of protein tetramerization [GO:1901090]; negatively regulates GO:0051262 Subtypes: negative regulation of protein homotetramerization [GO:1901094]